{
  "term_label": "Unknown cellular component",
  "term_id": "UNKNOWN:0003",
  "gene": "UniProtKB:Q9NQ03",
  "gene_symbol": "SCRT2",
  "gene_name": "Transcriptional repressor scratch 2"
}